{
  "gene": "UniProtKB:P01597",
  "term_id": "GO:0019814",
  "gene_name": "Immunoglobulin kappa variable 1-39",
  "gene_symbol": "IGKV1-39",
  "term_label": "immunoglobulin complex"
}